{
  "gene_symbol": "COL4A5",
  "gene": "UniProtKB:P29400",
  "gene_name": "Collagen alpha-5(IV) chain",
  "term_id": "GO:0030020",
  "term_label": "extracellular matrix structural constituent conferring tensile strength"
}